regulation of fungal-type cell wall organization [GO:0060237] (biological process) Also known as: regulation of fungal-type cell wall organisation, regulation of fungal-type cell wall organization and biogenesis Definition: Any process that modulates the rate, frequency or extent of the formation, arrangement of constituent parts, or disassembly of the fungal-type cell wall. Relationships: is a type of regulation of cellular component organization [GO:0051128]; is a type of regulation of cell wall organization or biogenesis [GO:1903338]; RO_0002211 fungal-type cell wall organization [GO:0031505] Sources: GOC:dph, GOC:tb